{
  "term_label": "RNA lariat debranching enzyme activity",
  "gene": "UniProtKB:Q9UK59",
  "gene_symbol": "DBR1",
  "gene_name": "Lariat debranching enzyme",
  "term_id": "GO:0008419"
}